caspase binding [GO:0089720] (molecular function) Definition: Binding to a caspase family protein. Sources: GOC:dos, GOC:ha Relationships: is a type of protease binding [GO:0002020]